{
  "gene": "UniProtKB:Q12983",
  "gene_name": "BCL2_adenovirus E1B 19 kDa protein-interacting protein 3",
  "term_id": "GO:0005783",
  "gene_symbol": "BNIP3",
  "term_label": "endoplasmic reticulum"
}